6G-fructosyltransferase activity [GO:0033841] (molecular function) Sources: EC:2.4.1.243 Relationships: is a type of fructosyltransferase activity [GO:0050738] Definition: Catalysis of the reaction: [1-beta-D-fructofuranosyl-(2->1)-]m+1 alpha-D-glucopyranoside + [1-beta-D-fructofuranosyl-(2->1)-]n+1 alpha-D-glucopyranoside = [1-beta-D-fructofuranosyl-(2->1)-]m alpha-D-glucopyranoside + [1-beta-D-fructofuranosyl-(2->1)-]n+1 beta-D-fructofuranosyl-(2->6)-alpha-D-glucopyranoside (m > 0; n >= 0). Also known as: 1F-oligo[beta-D-fructofuranosyl-(2->1)-]sucrose 6G-beta-D-fructotransferase activity, 6G-FFT, 6G-FT, 6G-fructotransferase activity, fructan:fructan 6G-fructosyltransferase activity